{
  "gene_symbol": "WHAMM",
  "gene_name": "WASP homolog-associated protein with actin, membranes and microtubules",
  "term_label": "endoplasmic reticulum to Golgi vesicle-mediated transport",
  "term_id": "GO:0006888",
  "gene": "UniProtKB:Q8TF30"
}